{
  "term_id": "UNKNOWN:0002",
  "term_label": "Unknown biological process",
  "gene_name": "Transmembrane protein 185B",
  "gene_symbol": "TMEM185B",
  "gene": "UniProtKB:Q9H7F4"
}